{
  "term_label": "Golgi membrane",
  "gene_symbol": "MGAT2",
  "term_id": "GO:0000139",
  "gene": "UniProtKB:Q10469",
  "gene_name": "Alpha-1,6-mannosyl-glycoprotein 2-beta-N-acetylglucosaminyltransferase"
}